{
  "term_label": "ubiquitin-like ligase-substrate adaptor activity",
  "gene_name": "Kelch-like protein 13",
  "term_id": "GO:1990756",
  "gene_symbol": "KLHL13",
  "gene": "UniProtKB:Q9P2N7"
}